{
  "gene_symbol": "TMTC3",
  "gene_name": "Protein O-mannosyl-transferase TMTC3",
  "gene": "UniProtKB:Q6ZXV5",
  "term_label": "protein O-linked glycosylation via mannose",
  "term_id": "GO:0035269"
}